{
  "term_id": "UNKNOWN:0003",
  "gene_symbol": "GFI1",
  "gene_name": "Zinc finger protein Gfi-1",
  "gene": "UniProtKB:Q99684",
  "term_label": "Unknown cellular component"
}